{
  "gene_symbol": "TRAV8-1",
  "gene_name": "T cell receptor alpha variable 8-1",
  "term_id": "GO:0019814",
  "term_label": "immunoglobulin complex",
  "gene": "UniProtKB:A0A0A6YYK1"
}